phosphatidylethanolamine-sterol O-acyltransferase activity [GO:0080095] (molecular function) References: PMID:16020547 Relationships: is a type of O-acyltransferase activity [GO:0008374] Definition: Catalysis of the reaction: a phosphatidylethanolamine + a sterol = a sterol ester + a lysophosphatidylethanolamine.